light-independent chlorophyll biosynthetic process [GO:0036068] (biological process) Relationships: is a type of chlorophyll biosynthetic process [GO:0015995] Definition: The chemical reactions and pathways resulting in the formation of chlorophyll, any compound of magnesium complexed in a porphyrin (tetrapyrrole) ring and which functions as a photosynthetic pigment, from less complex precursors, which occur in the absence of light. Also known as: light independent chlorophyll biosynthetic process, light-independent chlorophyll anabolism, light-independent chlorophyll biosynthesis, light-independent chlorophyll formation, light-independent chlorophyll synthesis Subtypes: light-independent bacteriochlorophyll biosynthetic process [GO:0036070] References: PMID:12242396 Sources: GOC:yaf